D-glucuronate transmembrane transport [GO:0042874] (biological process) Definition: The process in which D-glucuronate, the D-enantiomer of glucuronate, is transported across a lipid bilayer, from one side of a membrane to the other. Relationships: is a type of glucuronate transmembrane transport [GO:0015738] Sources: GOC:jl, GOC:jsg, GOC:mah Also known as: D-glucuronate transport